{
  "term_label": "Unknown cellular component",
  "term_id": "UNKNOWN:0003",
  "gene": "UniProtKB:Q7Z2K6",
  "gene_symbol": "ERMP1",
  "gene_name": "Endoplasmic reticulum metallopeptidase 1"
}